store-operated calcium channel activity [GO:0015279] (molecular function) Definition: A ligand-gated ion channel activity which transports calcium in response to emptying of intracellular calcium stores. Relationships: is a type of calcium channel activity [GO:0005262] References: PMID:15788710 Sources: GOC:dph, GOC:tb Regulation: RO_0002211 by regulation of store-operated calcium channel activity [GO:1901339]; negatively regulated by GO:1901340; positively regulated by GO:1901341